{
  "gene_symbol": "CDK17",
  "term_label": "cytoplasm",
  "gene": "UniProtKB:Q00537",
  "term_id": "GO:0005737",
  "gene_name": "Cyclin-dependent kinase 17"
}